{
  "gene_name": "CD40 ligand",
  "term_id": "GO:2001238",
  "gene": "UniProtKB:P29965",
  "gene_symbol": "CD40LG",
  "term_label": "positive regulation of extrinsic apoptotic signaling pathway"
}